{
  "gene": "UniProtKB:Q9H936",
  "gene_symbol": "SLC25A22",
  "term_label": "L-aspartate transmembrane transporter activity",
  "term_id": "GO:0015183",
  "gene_name": "Mitochondrial glutamate carrier 1"
}